{
  "gene_symbol": "LBP",
  "term_label": "extracellular space",
  "gene": "UniProtKB:P18428",
  "gene_name": "Lipopolysaccharide-binding protein",
  "term_id": "GO:0005615"
}